{
  "term_id": "GO:0003713",
  "term_label": "transcription coactivator activity",
  "gene_symbol": "MTA3",
  "gene": "UniProtKB:Q9BTC8",
  "gene_name": "Metastasis-associated protein MTA3"
}